{
  "term_id": "UNKNOWN:0002",
  "gene": "UniProtKB:Q9UPR6",
  "gene_name": "Zinc finger RNA-binding protein 2",
  "term_label": "Unknown biological process",
  "gene_symbol": "ZFR2"
}